{
  "gene_name": "Receptor-type tyrosine-protein kinase FLT3",
  "gene_symbol": "FLT3",
  "term_label": "B cell differentiation",
  "gene": "UniProtKB:P36888",
  "term_id": "GO:0030183"
}